{
  "term_label": "Unknown molecular function",
  "gene_symbol": "SCYGR2",
  "gene_name": "Small cysteine and glycine repeat-containing protein 2",
  "term_id": "UNKNOWN:0001",
  "gene": "UniProtKB:A0A286YFB4"
}